{
  "gene_symbol": "CHD3",
  "gene_name": "Chromodomain-helicase-DNA-binding protein 3",
  "term_id": "GO:0003677",
  "gene": "UniProtKB:Q12873",
  "term_label": "DNA binding"
}